{
  "gene_name": "Circadian locomoter output cycles protein kaput",
  "term_id": "GO:0070888",
  "term_label": "E-box binding",
  "gene": "UniProtKB:O15516",
  "gene_symbol": "CLOCK"
}